{
  "term_label": "microtubule organizing center",
  "gene": "UniProtKB:Q6ZN84",
  "gene_symbol": "CCDC81",
  "gene_name": "Coiled-coil domain-containing protein 81",
  "term_id": "GO:0005815"
}